CURI complex [GO:0032545] (CC) Definition: A protein complex that is involved in the transcription of ribosomal genes. In Saccharomyces this complex consists of Ckb2p, Utp22p, Rrp7p and Ifh1p. References: PMID:17452446 Relationships: is a type of GO:0140513